{
  "gene_name": "Chromodomain-helicase-DNA-binding protein 8",
  "term_id": "GO:0042393",
  "gene_symbol": "CHD8",
  "term_label": "histone binding",
  "gene": "UniProtKB:Q9HCK8"
}